3alpha,7alpha,12alpha-trihydroxy-5beta-cholest-24-enoyl-CoA hydratase activity [GO:0033989] (molecular function) Sources: EC:4.2.1.107 Relationships: is_a hydro-lyase activity [GO:0016836] Also known as: D-3-hydroxyacyl-CoA dehydratase activity, (24R,25R)-3alpha,7alpha,12alpha,24-tetrahydroxy-5beta-cholestanoyl-CoA hydro-lyase [(24E)-3alpha,7alpha,12alpha-trihydroxy-5beta-cholest-24-enoyl-CoA-forming] activity, (24R,25R)-3alpha,7alpha,12alpha,24-tetrahydroxy-5beta-cholestanoyl-CoA hydro-lyase activity, 46 kDa hydratase 2 activity Definition: Catalysis of the reaction: (24R,25R)-3alpha,7alpha,12alpha,24-tetrahydroxy-5beta-cholestanoyl-CoA = (24E)-3alpha,7alpha,12alpha-trihydroxy-5beta-cholest-24-enoyl-CoA + H2O.